{
  "gene_symbol": "TBX18",
  "term_id": "GO:0005634",
  "gene": "UniProtKB:O95935",
  "term_label": "nucleus",
  "gene_name": "T-box transcription factor TBX18"
}